phylloquinone catabolic process [GO:0042376] (biological process) Definition: The chemical reactions and pathways resulting in the breakdown of phylloquinone, vitamin K1, a quinone-derived compound synthesized by green plants. Also known as: phylloquinone breakdown, phylloquinone catabolism, phylloquinone degradation, phytomenadione catabolic process, phytomenadione catabolism, phytonadione catabolic process, phytonadione catabolism, phytylmenaquinone catabolic process, phytylmenaquinone catabolism, vitamin K1 catabolic process, vitamin K1 catabolism Relationships: is a type of vitamin K catabolic process [GO:0042377] References: PMID:27337968 Sources: GOC:jl, https://doi.org/10.1016/B978-0-12-385853-5.00001-5